{
  "term_label": "proteasome-mediated ubiquitin-dependent protein catabolic process",
  "gene_symbol": "KLHL13",
  "gene": "UniProtKB:Q9P2N7",
  "term_id": "GO:0043161",
  "gene_name": "Kelch-like protein 13"
}